L-tryptophan decarboxylase activity [GO:0036469] (molecular function) Definition: Catalysis of the reaction: L-tryptophan + H+ = CO2 + tryptamine. Sources: GOC:PARL, GOC:bf, RHEA:30339 Relationships: is a type of aromatic-L-amino-acid decarboxylase activity [GO:0004058]